{
  "gene_symbol": "AMMECR1",
  "term_id": "UNKNOWN:0001",
  "gene": "UniProtKB:Q9Y4X0",
  "term_label": "Unknown molecular function",
  "gene_name": "Nuclear protein AMMECR1"
}